regulation of Fc-gamma receptor signaling pathway involved in phagocytosis [GO:1905449] (biological process) Definition: Any process that modulates the frequency, rate or extent of Fc-gamma receptor signaling pathway involved in phagocytosis. Subtypes: negative regulation of Fc-gamma receptor signaling pathway involved in phagocytosis [GO:1905450], positive regulation of Fc-gamma receptor signaling pathway involved in phagocytosis [GO:1905451] Relationships: is_a regulation of immune effector process [GO:0002697]; is a type of GO:0060368; regulates Fc-gamma receptor signaling pathway involved in phagocytosis [GO:0038096] Also known as: regulation of Fc gamma receptor-dependent phagocytosis, regulation of Fc-gamma receptor signalling pathway involved in phagocytosis, regulation of Fcgamma receptor-mediated phagocytosis, regulation of IgG-mediated phagocytosis References: PMID:18832707 Sources: GOC:TermGenie, GO_REF:0000058